{
  "gene": "UniProtKB:O95377",
  "gene_name": "Gap junction beta-5 protein",
  "gene_symbol": "GJB5",
  "term_id": "GO:0005922",
  "term_label": "connexin complex"
}